regulation of monocyte antigen processing and presentation [GO:0002613] (biological process) Relationships: is a type of GO:0002577; regulates monocyte antigen processing and presentation [GO:0002471] Subtypes: negative regulation of monocyte antigen processing and presentation [GO:0002614], GO:0002615 Definition: Any process that modulates the frequency, rate, or extent of monocyte antigen processing and presentation. Sources: GOC:add